{
  "gene_name": "Neural proliferation differentiation and control protein 1",
  "term_id": "UNKNOWN:0001",
  "term_label": "Unknown molecular function",
  "gene": "UniProtKB:Q9NQX5",
  "gene_symbol": "NPDC1"
}